{
  "gene_name": "Teashirt homolog 3",
  "term_label": "regulation of transcription by RNA polymerase II",
  "term_id": "GO:0006357",
  "gene": "UniProtKB:Q63HK5",
  "gene_symbol": "TSHZ3"
}